negative regulation of kainate selective glutamate receptor signaling pathway [GO:0106427] (biological process) Relationships: is a type of negative regulation of biological process [GO:0048519]; is a type of regulation of kainate selective glutamate receptor signaling pathway [GO:0106426]; negatively regulates regulation of kainate selective glutamate receptor signaling pathway [GO:0106426] References: PMID:12597860 Definition: Any process that stops, prevents or reduces the frequency, rate or extent of the kainate selective glutamate receptor signaling pathway.